{
  "gene_symbol": "POLR2H",
  "gene_name": "DNA-directed RNA polymerases I, II, and III subunit RPABC3",
  "term_label": "DNA-directed RNA polymerase activity",
  "gene": "UniProtKB:P52434",
  "term_id": "GO:0003899"
}